{
  "term_label": "chemical synaptic transmission",
  "gene_symbol": "HTR2C",
  "gene": "UniProtKB:P28335",
  "gene_name": "5-hydroxytryptamine receptor 2C",
  "term_id": "GO:0007268"
}